oocyte anterior/posterior axis specification [GO:0007314] (biological process) Definition: Polarization of the oocyte along its anterior-posterior axis. An example of this is found in Drosophila melanogaster. Relationships: is a type of oocyte axis specification [GO:0007309]; is a type of anterior/posterior axis specification [GO:0009948]; is part of maternal determination of anterior/posterior axis, embryo [GO:0008358] Sources: GOC:dph, GOC:mtg_sensu, GOC:tb, ISBN:0879694238 Also known as: oocyte anterior/posterior axis determination